cell wall [GO:0005618] (cellular component) Note: Not to be used for manual annotation. Please choose a more specific term: for bacteria, annotate to GO:0009274; peptidoglycan-based cell wall, for plants: annotate to GO:0009505 ; plant-type cell wall, for fungi: GO:0009277 ; fungal-type cell wall, and for archae, use GO:0030115 S-layer (see PMID:31214995). References: PMID:15134259 Sources: GOC:giardia, ISBN:0198547684, Wikipedia:Microbial_cyst Relationships: is a type of external encapsulating structure [GO:0030312] Subtypes: peptidoglycan-based cell wall [GO:0009274], fungal-type cell wall [GO:0009277], plant-type cell wall [GO:0009505], spore wall [GO:0031160], cyst wall [GO:0097570] Definition: The rigid or semi-rigid envelope lying outside the cell membrane of plant, fungal, most prokaryotic cells and some protozoan parasites, maintaining their shape and protecting them from osmotic lysis. In plants it is made of cellulose and, often, lignin; in fungi it is composed largely of polysaccharides; in bacteria it is composed of peptidoglycan; in protozoan parasites such as Giardia species, it's made of carbohydrates and proteins.